{
  "gene_symbol": "ZNF574",
  "gene": "UniProtKB:Q6ZN55",
  "term_id": "GO:0005634",
  "term_label": "nucleus",
  "gene_name": "Zinc finger protein 574"
}